vitamin B6 transport [GO:0031919] (biological process) Subtypes: GO:0031920, pyridoxal phosphate transport [GO:0031921], pyridoxamine transport [GO:0031922], pyridoxine transport [GO:0031923] Sources: GOC:mah Relationships: is a type of vitamin transport [GO:0051180]; is a type of nitrogen compound transport [GO:0071705] Definition: The directed movement of any of the vitamin B6 compounds -- pyridoxal, pyridoxamine and pyridoxine and the active form, pyridoxal phosphate -- into, out of or within a cell, or between cells, by means of some agent such as a transporter or pore.